{
  "gene_symbol": "DOK3",
  "gene_name": "Docking protein 3",
  "term_id": "GO:0007265",
  "term_label": "Ras protein signal transduction",
  "gene": "UniProtKB:Q7L591"
}